molecular function activator activity [GO:0140677] (molecular function) Definition: A molecular function regulator that activates or increases the activity of its target via non-covalent binding that does not result in covalent modification to the target. Subtypes: actin severing activator activity [GO:0000513], ATPase activator activity [GO:0001671], GO:0008047, signaling receptor activator activity [GO:0030546], transcription regulator activator activity [GO:0140537], cytoskeletal motor activator activity [GO:0140660], GO:0141109 Note: This term should only be used in cases when the regulator directly interacts with the enzyme, but does not result in a covalent modification. Sources: GOC:curators Relationships: is a type of molecular function regulator activity [GO:0098772]